{
  "term_id": "GO:0055038",
  "gene_name": "Rab11 family-interacting protein 3",
  "gene": "UniProtKB:O75154",
  "term_label": "recycling endosome membrane",
  "gene_symbol": "RAB11FIP3"
}